optokinetic behavior [GO:0007634] (biological process) Definition: The behavior of an organism pertaining to movement of the eyes and of objects in the visual field, as in nystagmus. Also known as: optokinetic behaviour Subtypes: optomotor response [GO:0071632] Relationships: is a type of GO:0007632 Sources: GOC:jid, GOC:pr